{
  "term_id": "UNKNOWN:0002",
  "gene_symbol": "ZCCHC14",
  "term_label": "Unknown biological process",
  "gene_name": "Zinc finger CCHC domain-containing protein 14",
  "gene": "UniProtKB:Q8WYQ9"
}